{
  "term_label": "intraciliary transport particle B binding",
  "term_id": "GO:0120170",
  "gene_name": "Intraflagellar transport protein 70B",
  "gene": "UniProtKB:Q8N4P2",
  "gene_symbol": "IFT70B"
}